{
  "gene_symbol": "DIP2B",
  "term_id": "UNKNOWN:0003",
  "gene_name": "Disco-interacting protein 2 homolog B",
  "term_label": "Unknown cellular component",
  "gene": "UniProtKB:Q9P265"
}